(4S)-limonene synthase activity [GO:0050552] (molecular function) Definition: Catalysis of the reaction: geranyl diphosphate = (4S)-limonene + diphosphate. Relationships: is a type of terpene synthase activity [GO:0010333] Sources: EC:4.2.3.16, MetaCyc:4.2.3.16-RXN Also known as: (-)-(4S)-limonene synthase activity, 4S-(-)-limonene synthase activity, geranyl-diphosphate diphosphate-lyase [cyclizing, (-)-(4S)-limonene-forming], geranyldiphosphate diphosphate lyase (limonene forming), geranyldiphosphate diphosphate lyase [cyclizing, (4S)-limonene-forming]